{
  "gene_symbol": "ACTB",
  "gene": "UniProtKB:P60709",
  "term_label": "structural constituent of postsynaptic actin cytoskeleton",
  "term_id": "GO:0098973",
  "gene_name": "Actin, cytoplasmic 1"
}